{
  "gene_name": "Zinc finger protein 80",
  "term_label": "RNA polymerase II transcription regulatory region sequence-specific DNA binding",
  "gene_symbol": "ZNF80",
  "term_id": "GO:0000977",
  "gene": "UniProtKB:P51504"
}